{
  "term_id": "GO:0030276",
  "gene_name": "Putative tyrosine-protein phosphatase auxilin",
  "gene": "UniProtKB:O75061",
  "term_label": "clathrin binding",
  "gene_symbol": "DNAJC6"
}